{
  "gene_name": "Transcription factor TFIIIB component B'' homolog",
  "term_label": "RNA polymerase III preinitiation complex assembly",
  "gene": "UniProtKB:A6H8Y1",
  "gene_symbol": "BDP1",
  "term_id": "GO:0070898"
}